proteasome core complex [GO:0005839] (cellular component) Definition: A multisubunit barrel shaped endoprotease complex, which is the core of the proteasome complex. Relationships: is a type of GO:0140535; is a type of catalytic complex [GO:1902494]; is part of proteasome complex [GO:0000502] Also known as: macropain, 20S core complex, 20S proteasome, PA28gamma-20S proteasome References: PMID:10806206 Sources: GOC:rb Subtypes: nuclear proteasome core complex [GO:0031601], cytosolic proteasome core complex [GO:0031603]